{
  "gene_name": "Transcription factor Spi-B",
  "term_label": "DNA-binding transcription factor activity, RNA polymerase II-specific",
  "gene": "UniProtKB:Q01892",
  "term_id": "GO:0000981",
  "gene_symbol": "SPIB"
}